{
  "gene": "UniProtKB:A0A087WZ39",
  "gene_name": "T cell receptor beta variable 15 (Fragment)",
  "gene_symbol": "TRBV15",
  "term_id": "UNKNOWN:0001",
  "term_label": "Unknown molecular function"
}